{
  "term_id": "GO:0048015",
  "gene_symbol": "PLCG2",
  "term_label": "phosphatidylinositol-mediated signaling",
  "gene": "UniProtKB:P16885",
  "gene_name": "1-phosphatidylinositol 4,5-bisphosphate phosphodiesterase gamma-2"
}